{
  "term_id": "GO:0006357",
  "gene": "UniProtKB:O00110",
  "term_label": "regulation of transcription by RNA polymerase II",
  "gene_symbol": "OVOL3",
  "gene_name": "Putative transcription factor ovo-like protein 3"
}